S-malonyltransferase activity [GO:0016419] (molecular function) Sources: GOC:ai Relationships: is a type of GO:0016417; is a type of malonyltransferase activity [GO:0016420] Definition: Catalysis of the transfer of a malonyl group to a sulfur atom on the acceptor molecule. Subtypes: GO:0004314